TFIIH-class transcription factor complex binding [GO:0001097] (molecular function) Relationships: is a type of RNA polymerase II general transcription initiation factor binding [GO:0001091]; is a type of protein-containing complex binding [GO:0044877] Also known as: TFIIH-class transcription factor binding References: PMID:16858867 Sources: GOC:krc Definition: Binding to a general RNA polymerase II transcription factor belonging to the TFIIH complex, one of the factors involved in formation of the preinitiation complex (PIC) by RNA polymerase II.